{
  "gene_symbol": "MYH8",
  "gene": "UniProtKB:P13535",
  "gene_name": "Myosin-8",
  "term_id": "GO:0000146",
  "term_label": "microfilament motor activity"
}